{
  "gene_symbol": "KRT86",
  "gene": "UniProtKB:O43790",
  "gene_name": "Keratin, type II cuticular Hb6",
  "term_label": "structural constituent of skin epidermis",
  "term_id": "GO:0030280"
}